{
  "gene_name": "Elongation factor 1-beta",
  "gene": "UniProtKB:P24534",
  "term_label": "guanyl-nucleotide exchange factor activity",
  "term_id": "GO:0005085",
  "gene_symbol": "EEF1B2"
}